{
  "term_id": "GO:0006749",
  "term_label": "glutathione metabolic process",
  "gene": "UniProtKB:O43708",
  "gene_symbol": "GSTZ1",
  "gene_name": "Maleylacetoacetate isomerase"
}